(S)-2-hydroxy-fatty acid dehydrogenase activity [GO:0047050] (molecular function) Definition: Catalysis of the reaction: (S)-2-hydroxystearate + NAD+ = 2-oxostearate + H+ + NADH. Relationships: is a type of oxidoreductase activity, acting on the CH-OH group of donors, NAD or NADP as acceptor [GO:0016616] Also known as: 2-hydroxy fatty acid oxidase, (S)-2-hydroxy-fatty-acid dehydrogenase activity, (S)-2-hydroxystearate:NAD+ oxidoreductase activity, L-2-hydroxy fatty acid dehydrogenase activity, dehydrogenase, L-2-hydroxy fatty acid Sources: EC:1.1.1.99, RHEA:11384